{
  "term_id": "GO:0006909",
  "gene_name": "5'-3' exonuclease PLD4",
  "term_label": "phagocytosis",
  "gene": "UniProtKB:Q96BZ4",
  "gene_symbol": "PLD4"
}